{
  "gene": "UniProtKB:Q96HC4",
  "term_id": "GO:0030036",
  "term_label": "actin cytoskeleton organization",
  "gene_name": "PDZ and LIM domain protein 5",
  "gene_symbol": "PDLIM5"
}